{
  "gene_symbol": "SHH",
  "gene": "UniProtKB:Q15465",
  "gene_name": "Sonic hedgehog protein",
  "term_id": "GO:0005615",
  "term_label": "extracellular space"
}